{
  "gene": "UniProtKB:A6NMD0",
  "gene_symbol": "IFITM10",
  "gene_name": "Interferon-induced transmembrane protein 10",
  "term_id": "UNKNOWN:0002",
  "term_label": "Unknown biological process"
}